{
  "term_label": "Unknown biological process",
  "gene_symbol": "CMTM2",
  "term_id": "UNKNOWN:0002",
  "gene": "UniProtKB:Q8TAZ6",
  "gene_name": "CKLF-like MARVEL transmembrane domain-containing protein 2"
}